{
  "gene_symbol": "CLEC3B",
  "gene_name": "Tetranectin",
  "term_label": "bone mineralization",
  "gene": "UniProtKB:P05452",
  "term_id": "GO:0030282"
}